{
  "gene_symbol": "ART4",
  "gene": "UniProtKB:Q93070",
  "gene_name": "Ecto-ADP-ribosyltransferase 4",
  "term_id": "GO:0003950",
  "term_label": "NAD+ poly-ADP-ribosyltransferase activity"
}